negative regulation of methanofuran biosynthetic process [GO:1900352] (biological process) Definition: Any process that stops, prevents or reduces the frequency, rate or extent of methanofuran biosynthetic process. Relationships: is a type of negative regulation of biosynthetic process [GO:0009890]; is a type of regulation of methanofuran biosynthetic process [GO:1900351]; negatively regulates methanofuran biosynthetic process [GO:2001120] Also known as: down regulation of methanofuran biosynthesis, down regulation of methanofuran biosynthetic process, down-regulation of methanofuran biosynthesis, down-regulation of methanofuran biosynthetic process, downregulation of methanofuran biosynthesis, downregulation of methanofuran biosynthetic process, inhibition of methanofuran biosynthesis, negative regulation of methanofuran biosynthesis, inhibition of methanofuran biosynthetic process Sources: GOC:TermGenie, GOC:mengo_curators